{
  "gene_symbol": "SYNE1",
  "term_id": "GO:0051642",
  "term_label": "centrosome localization",
  "gene": "UniProtKB:Q8NF91",
  "gene_name": "Nesprin-1"
}